{
  "gene_name": "Large ribosomal subunit protein eL43",
  "term_id": "UNKNOWN:0001",
  "gene_symbol": "RPL37A",
  "gene": "UniProtKB:P61513",
  "term_label": "Unknown molecular function"
}